{
  "gene_symbol": "SLC2A1",
  "term_id": "GO:0046323",
  "term_label": "D-glucose import",
  "gene_name": "Solute carrier family 2, facilitated glucose transporter member 1",
  "gene": "UniProtKB:P11166"
}